{
  "term_label": "cone photoreceptor outer segment",
  "gene_name": "Guanylyl cyclase-activating protein 2",
  "gene_symbol": "GUCA1B",
  "gene": "UniProtKB:Q9UMX6",
  "term_id": "GO:0120199"
}